inner plaque of spindle pole body [GO:0005822] (CC) Sources: ISBN:0879693568 Definition: One of three laminate structures that form the spindle pole body; the inner plaque is in the nucleus. Relationships: is a type of GO:0110165; BFO_0000050 spindle pole body [GO:0005816] Subtypes: inner plaque of mitotic spindle pole body [GO:0061497]